{
  "gene_symbol": "TSNAX",
  "term_label": "RNA binding",
  "term_id": "GO:0003723",
  "gene": "UniProtKB:Q99598",
  "gene_name": "Translin-associated protein X"
}